{
  "term_id": "GO:0004984",
  "gene_symbol": "OR2A2",
  "gene": "UniProtKB:Q6IF42",
  "gene_name": "Olfactory receptor 2A2",
  "term_label": "olfactory receptor activity"
}